{
  "term_id": "GO:0006357",
  "gene_symbol": "ZNF396",
  "gene_name": "Zinc finger protein 396",
  "term_label": "regulation of transcription by RNA polymerase II",
  "gene": "UniProtKB:Q96N95"
}